{
  "gene_symbol": "KCNG4",
  "term_id": "GO:0015459",
  "gene": "UniProtKB:Q8TDN1",
  "gene_name": "Potassium voltage-gated channel subfamily G member 4",
  "term_label": "potassium channel regulator activity"
}